FHL2-CREB complex [GO:0034980] (cellular component) Definition: A protein complex that contains CREB and FHL2, and is involved in transcriptional regulation. References: PMID:11046156 Relationships: is a type of DNA helicase complex [GO:0033202]; is_a nuclear protein-containing complex [GO:0140513]